{
  "gene_symbol": "PKDREJ",
  "gene": "UniProtKB:Q9NTG1",
  "term_label": "membrane",
  "term_id": "GO:0016020",
  "gene_name": "Polycystin family receptor for egg jelly"
}